{
  "term_id": "GO:0005886",
  "term_label": "plasma membrane",
  "gene_symbol": "PLPPR2",
  "gene": "UniProtKB:Q96GM1",
  "gene_name": "Phospholipid phosphatase-related protein type 2"
}